TRAM-dependent toll-like receptor 4 signaling pathway [GO:0035669] (biological process) Relationships: is a type of toll-like receptor 4 signaling pathway [GO:0034142]; is a type of GO:0035668 References: PMID:14556004, PMID:18297073 Sources: GOC:BHF Definition: The series of molecular signals initiated by a ligand binding to a toll-like receptor 4 where the TRAM adaptor mediates transduction of the signal. Toll-like 4 receptors are pattern recognition receptors that bind bacterial lipopolysaccharide (LPS) to initiate an innate immune response. Also known as: TRAM-dependent TLR4 signaling pathway, TRAM-dependent toll-like receptor 4 signalling pathway